response to methanol [GO:0033986] (biological process) Sources: GOC:sl Relationships: is a type of GO:0097305 Definition: Any process that results in a change in state or activity of a cell or an organism (in terms of movement, secretion, enzyme production, gene expression, etc.) as a result of a methanol stimulus. Subtypes: cellular response to methanol [GO:0071405]